{
  "gene_symbol": "CHRNA7",
  "term_label": "acetylcholine-gated channel complex",
  "term_id": "GO:0005892",
  "gene_name": "Neuronal acetylcholine receptor subunit alpha-7",
  "gene": "UniProtKB:P36544"
}